{
  "gene_name": "Uncharacterized protein KIAA1755",
  "term_id": "GO:0005737",
  "gene": "UniProtKB:Q5JYT7",
  "term_label": "cytoplasm",
  "gene_symbol": "KIAA1755"
}